{
  "term_label": "chromatin remodeling",
  "gene": "UniProtKB:A0A1W2PPD8",
  "gene_name": "Probable lysine-specific demethylase 4F",
  "term_id": "GO:0006338",
  "gene_symbol": "KDM4F"
}